{
  "term_label": "axon",
  "gene_symbol": "PRPH",
  "term_id": "GO:0030424",
  "gene_name": "Peripherin",
  "gene": "UniProtKB:P41219"
}